{
  "gene_symbol": "TMEM67",
  "term_label": "Unknown molecular function",
  "term_id": "UNKNOWN:0001",
  "gene_name": "Meckelin",
  "gene": "UniProtKB:Q5HYA8"
}